interphase microtubule organizing center [GO:0031021] (cellular component) Also known as: iMTOC, interphase MTOC, interphase microtubule organising center Relationships: is a type of GO:0005815 Definition: A microtubule organizing center found in interphase cells, which organize a longitudinal array of three to five MT bundles from the nuclear envelope during interphase. Each MT bundle is composed of two to seven MTs arranged in an antiparallel configuration, with the dynamic MT plus ends extending toward the cell tips and stable minus ends near the nucleus. References: PMID:15068790